citrate metabolic process [GO:0006101] (biological process) Also known as: citrate metabolism Definition: The chemical reactions and pathways involving citrate, 2-hydroxy-1,2,3-propanetricarboxylate. Citrate is widely distributed in nature and is an important intermediate in the TCA cycle and the glyoxylate cycle. Relationships: is a type of tricarboxylic acid metabolic process [GO:0072350] Subtypes: citrate catabolic process to diacetyl [GO:0019651] Sources: ISBN:0198506732